{
  "gene_name": "Uncharacterized protein C2orf27A",
  "gene_symbol": "C2orf27A",
  "gene": "UniProtKB:P0DPF5",
  "term_label": "Unknown biological process",
  "term_id": "UNKNOWN:0002"
}